{
  "term_label": "glycolipid biosynthetic process",
  "term_id": "GO:0009247",
  "gene_symbol": "ST3GAL4",
  "gene": "UniProtKB:Q11206",
  "gene_name": "CMP-N-acetylneuraminate-beta-galactosamide-alpha-2,3-sialyltransferase 4"
}